regulation of type II interferon-mediated signaling pathway [GO:0060334] (biological process) Relationships: is a type of regulation of cytokine-mediated signaling pathway [GO:0001959]; is a type of GO:0060330; regulates GO:0060333 Subtypes: positive regulation of type II interferon-mediated signaling pathway [GO:0060335], negative regulation of type II interferon-mediated signaling pathway [GO:0060336] Also known as: regulation of type II IFN-mediated signaling pathway, regulation of immune interferon signaling pathway, regulation of interferon-gamma-mediated signaling pathway, regulation of interferon-gamma-mediated signalling pathway, regulation of gamma-interferon-mediated signaling pathway Sources: GOC:dph Definition: Any process that modulates the rate, frequency or extent of an interferon-gamma-mediated signaling pathway.